{
  "term_id": "UNKNOWN:0003",
  "gene_symbol": "RBM42",
  "gene": "UniProtKB:Q9BTD8",
  "gene_name": "RNA-binding protein 42",
  "term_label": "Unknown cellular component"
}